{
  "gene": "UniProtKB:P31941",
  "gene_name": "DNA dC-dU-editing enzyme APOBEC-3A",
  "term_label": "RNA binding",
  "gene_symbol": "APOBEC3A",
  "term_id": "GO:0003723"
}